{
  "gene_symbol": "VSIG2",
  "gene": "UniProtKB:Q96IQ7",
  "term_id": "UNKNOWN:0003",
  "term_label": "Unknown cellular component",
  "gene_name": "V-set and immunoglobulin domain-containing protein 2"
}